{
  "gene_name": "Multiple C2 and transmembrane domain-containing protein 1",
  "term_id": "GO:0030672",
  "gene": "UniProtKB:Q6DN14",
  "term_label": "synaptic vesicle membrane",
  "gene_symbol": "MCTP1"
}